positive regulation of somatic stem cell population maintenance [GO:1904674] (biological process) Definition: Any process that activates or increases the frequency, rate or extent of somatic stem cell population maintenance. Also known as: up regulation of somatic stem cell population maintenance, up-regulation of somatic stem cell population maintenance, upregulation of somatic stem cell population maintenance, activation of somatic stem cell population maintenance Subtypes: positive regulation of mesenchymal cell apoptotic process involved in nephron morphogenesis [GO:0072041] Relationships: is a type of positive regulation of stem cell population maintenance [GO:1902459]; is a type of regulation of somatic stem cell population maintenance [GO:1904672]; positively regulates somatic stem cell population maintenance [GO:0035019] References: PMID:19409607 Sources: GOC:BHF, GOC:BHF_miRNA, GOC:TermGenie, GOC:rph, GO_REF:0000058